endospore cortex [GO:0043595] (cellular component) Sources: GOC:mlg Relationships: is a type of cellular anatomical structure [GO:0110165]; is part of GO:0043591 Definition: A layer surrounding a bacterial endospore found inside the outer endospore membrane, but outside the membrane surrounding the endospore core. It consists of peptidoglycan of a different chemical nature than that found in vegetative cell walls which results in less cross-linking of peptidoglycan.